nucleophagy [GO:0044804] (biological process) Also known as: autophagy of nucleus, late nucleophagy, nucleus degradation References: PMID:24013549 Sources: GOC:autophagy, GOC:jl Definition: A form of autophagy, by which damaged or non-essential parts of the nucleus, or even an entire nucleus is degraded. Relationships: is a type of GO:0016236 Subtypes: piecemeal microautophagy of the nucleus [GO:0034727]